{
  "gene": "UniProtKB:A0A3B3IU46",
  "term_label": "mRNA capping enzyme complex",
  "term_id": "GO:0031533",
  "gene_symbol": "RAMACL",
  "gene_name": "RNA guanine-N7 methyltransferase-activating subunit-like protein"
}